{
  "gene": "UniProtKB:Q9H0A3",
  "term_id": "UNKNOWN:0001",
  "gene_symbol": "TMEM191A",
  "term_label": "Unknown molecular function",
  "gene_name": "Transmembrane protein 191A"
}